{
  "gene_name": "Testis-expressed protein 101",
  "term_label": "Unknown molecular function",
  "term_id": "UNKNOWN:0001",
  "gene_symbol": "TEX101",
  "gene": "UniProtKB:Q9BY14"
}